{
  "gene_name": "Doublesex- and mab-3-related transcription factor C2",
  "term_id": "UNKNOWN:0001",
  "gene": "UniProtKB:Q8IXT2",
  "term_label": "Unknown molecular function",
  "gene_symbol": "DMRTC2"
}